{
  "gene_name": "Kinesin-like protein KIF18B",
  "term_label": "cytoplasm",
  "gene": "UniProtKB:Q86Y91",
  "term_id": "GO:0005737",
  "gene_symbol": "KIF18B"
}